{
  "term_label": "nucleoplasm",
  "gene": "UniProtKB:Q99729",
  "gene_symbol": "HNRNPAB",
  "gene_name": "Heterogeneous nuclear ribonucleoprotein A_B",
  "term_id": "GO:0005654"
}